lung induction [GO:0060492] (biological process) Sources: GOC:dph Definition: The close range interaction of two or more cells or tissues that causes the cells of the foregut to change their fates and specify the development of the lung. Relationships: is a type of GO:0001759; is a type of GO:0045995; is a type of GO:0061046; positively regulates lung field specification [GO:0060424]